{
  "term_id": "GO:0000978",
  "gene_name": "Zinc finger protein 697",
  "gene_symbol": "ZNF697",
  "gene": "UniProtKB:Q5TEC3",
  "term_label": "RNA polymerase II cis-regulatory region sequence-specific DNA binding"
}